{
  "gene_name": "Diencephalon_mesencephalon homeobox protein 1",
  "term_label": "regulation of transcription by RNA polymerase II",
  "term_id": "GO:0006357",
  "gene_symbol": "DMBX1",
  "gene": "UniProtKB:Q8NFW5"
}